{
  "gene_symbol": "GSDMD",
  "term_id": "GO:0070269",
  "gene": "UniProtKB:P57764",
  "gene_name": "Gasdermin-D",
  "term_label": "pyroptotic inflammatory response"
}